{
  "term_label": "Unknown molecular function",
  "term_id": "UNKNOWN:0001",
  "gene": "UniProtKB:Q7Z304",
  "gene_symbol": "MAMDC2",
  "gene_name": "MAM domain-containing protein 2"
}